{
  "term_label": "cytoplasm",
  "gene_symbol": "LIN28A",
  "term_id": "GO:0005737",
  "gene_name": "Protein lin-28 homolog A",
  "gene": "UniProtKB:Q9H9Z2"
}